{
  "gene": "UniProtKB:Q9Y4D2",
  "gene_name": "Diacylglycerol lipase-alpha",
  "term_label": "arachidonate metabolic process",
  "gene_symbol": "DAGLA",
  "term_id": "GO:0019369"
}